{
  "term_id": "GO:0030154",
  "gene_symbol": "CDX2",
  "term_label": "cell differentiation",
  "gene": "UniProtKB:Q99626",
  "gene_name": "Homeobox protein CDX-2"
}